{
  "gene_name": "Antizyme inhibitor 2",
  "term_id": "GO:0042978",
  "gene_symbol": "AZIN2",
  "gene": "UniProtKB:Q96A70",
  "term_label": "ornithine decarboxylase activator activity"
}